{
  "term_id": "GO:0007520",
  "term_label": "myoblast fusion",
  "gene": "UniProtKB:Q92608",
  "gene_symbol": "DOCK2",
  "gene_name": "Dedicator of cytokinesis protein 2"
}